{
  "gene": "UniProtKB:Q16658",
  "gene_name": "Fascin",
  "term_label": "filopodium",
  "term_id": "GO:0030175",
  "gene_symbol": "FSCN1"
}